{
  "term_label": "nucleus",
  "gene": "UniProtKB:Q9NR33",
  "term_id": "GO:0005634",
  "gene_symbol": "POLE4",
  "gene_name": "DNA polymerase epsilon subunit 4"
}